{
  "gene_name": "Solute carrier family 15 member 3",
  "term_id": "GO:0071916",
  "term_label": "dipeptide transmembrane transporter activity",
  "gene_symbol": "SLC15A3",
  "gene": "UniProtKB:Q8IY34"
}